{
  "gene": "UniProtKB:Q9Y2W7",
  "term_id": "GO:0000122",
  "gene_symbol": "KCNIP3",
  "term_label": "negative regulation of transcription by RNA polymerase II",
  "gene_name": "Calsenilin"
}